heart rudiment involution [GO:0003320] (biological process) Sources: GOC:mtg_heart Relationships: is a type of morphogenesis of an epithelial fold involved in embryonic heart tube formation [GO:0003152] Definition: The inward folding of myocardial tissue derived from the right half of the heart rudiment that will form the future ventral part of the heart tube.